bipolar cellular bud site selection [GO:0007121] (biological process) Definition: The process of defining subsequent sites of bud emergence such that budding takes place at alternating poles of a budding cell. Relationships: is a type of cellular bud site selection [GO:0000282]; is a type of cell budding [GO:0007114] Sources: GOC:clt Also known as: bipolar budding, polar budding, bipolar bud site selection